{
  "gene_symbol": "ARMCX5",
  "term_label": "Unknown molecular function",
  "gene": "UniProtKB:Q6P1M9",
  "term_id": "UNKNOWN:0001",
  "gene_name": "Armadillo repeat-containing X-linked protein 5"
}